regulation of leukocyte differentiation [GO:1902105] (biological process) Relationships: is a type of regulation of hemopoiesis [GO:1903706]; regulates leukocyte differentiation [GO:0002521] Also known as: regulation of immune cell differentiation, regulation of leucocyte differentiation Sources: GOC:TermGenie, GOC:add Subtypes: regulation of myeloid leukocyte differentiation [GO:0002761], regulation of lymphocyte differentiation [GO:0045619], negative regulation of leukocyte differentiation [GO:1902106], GO:1902107, regulation of dendritic cell differentiation [GO:2001198] Definition: Any process that modulates the frequency, rate or extent of leukocyte differentiation.